L-tyrosine biosynthetic process [GO:0006571] (biological process) Also known as: tyrosine anabolism, tyrosine biosynthesis, tyrosine formation, tyrosine synthesis Relationships: is a type of GO:0006570; is a type of aromatic amino acid family biosynthetic process, prephenate pathway [GO:0009095]; is a type of GO:0170034; is a type of GO:0170038 Definition: The chemical reactions and pathways resulting in the formation of tyrosine, an aromatic amino acid, 2-amino-3-(4-hydroxyphenyl)propanoic acid. Subtypes: L-tyrosine biosynthetic process from chorismate via 4-hydroxyphenylpyruvate [GO:0019292], GO:0019293, L-tyrosine biosynthetic process from chorismate via L-arogenate [GO:0033584] Sources: GOC:sm